{
  "gene_name": "Sodium-dependent serotonin transporter",
  "term_label": "serotonin binding",
  "gene": "UniProtKB:P31645",
  "gene_symbol": "SLC6A4",
  "term_id": "GO:0051378"
}